{
  "gene_name": "Atypical chemokine receptor 2",
  "term_id": "GO:0016493",
  "gene_symbol": "ACKR2",
  "gene": "UniProtKB:O00590",
  "term_label": "C-C chemokine receptor activity"
}